{
  "term_id": "GO:0007160",
  "gene": "UniProtKB:P02675",
  "term_label": "cell-matrix adhesion",
  "gene_name": "Fibrinogen beta chain",
  "gene_symbol": "FGB"
}